{
  "term_label": "cytosol",
  "gene_name": "Carnosine N-methyltransferase",
  "gene": "UniProtKB:Q8N4J0",
  "term_id": "GO:0005829",
  "gene_symbol": "CARNMT1"
}